{
  "term_id": "GO:0044183",
  "term_label": "protein folding chaperone",
  "gene": "UniProtKB:P0DMV8",
  "gene_symbol": "HSPA1A",
  "gene_name": "Heat shock 70 kDa protein 1A"
}